{
  "term_id": "UNKNOWN:0001",
  "term_label": "Unknown molecular function",
  "gene_symbol": "TMEM185A",
  "gene_name": "Transmembrane protein 185A",
  "gene": "UniProtKB:Q8NFB2"
}